{
  "term_label": "Unknown biological process",
  "gene_name": "Dynein light chain 2, cytoplasmic",
  "gene": "UniProtKB:Q96FJ2",
  "term_id": "UNKNOWN:0002",
  "gene_symbol": "DYNLL2"
}